rRNA (guanosine-2'-O-)-methyltransferase activity [GO:0070039] (molecular function) Sources: GOC:imk, GOC:mah Relationships: is a type of rRNA (guanine) methyltransferase activity [GO:0016435]; is a type of RNA 2'-O-methyltransferase activity [GO:0062105]; is part of rRNA 2'-O-methylation [GO:0000451] Definition: Catalysis of the reaction: S-adenosyl-L-methionine + rRNA = S-adenosyl-L-homocysteine + rRNA containing 2'-O-methylguanosine.